type 2 vasoactive intestinal polypeptide receptor binding [GO:0031892] (molecular function) Relationships: is a type of GO:0031890 Sources: GOC:mah, GOC:nln Also known as: type 3 PACAP receptor binding, type 2 vasoactive intestinal polypeptide receptor ligand Definition: Binding to a type 2 vasoactive intestinal polypeptide receptor.